alpha2-beta1 integrin-CD47 complex [GO:0071084] (cellular component) Also known as: ITGA2-ITGB1-CD47 complex References: PMID:10397731 Relationships: is a type of GO:0098797 Definition: A protein complex that consists of an alpha2-beta1 integrin complex bound to the cell surface protein CD47.